{
  "term_id": "GO:0036064",
  "gene": "UniProtKB:O43805",
  "gene_name": "Microtubule nucleation factor SSNA1",
  "gene_symbol": "SSNA1",
  "term_label": "ciliary basal body"
}